{
  "term_label": "Unknown molecular function",
  "term_id": "UNKNOWN:0001",
  "gene_symbol": "STRA6",
  "gene_name": "Receptor for retinol uptake STRA6",
  "gene": "UniProtKB:Q9BX79"
}